{
  "term_id": "GO:0030198",
  "gene": "UniProtKB:O60882",
  "gene_symbol": "MMP20",
  "term_label": "extracellular matrix organization",
  "gene_name": "Matrix metalloproteinase-20"
}